inosine catabolic process [GO:0006148] (biological process) Sources: GOC:go_curators Definition: The chemical reactions and pathways resulting in the breakdown of inosine, hypoxanthine riboside, a nucleoside found free but not in combination in nucleic acids except in the anticodons of some tRNAs. Relationships: is a type of inosine metabolic process [GO:0046102]; is a type of purine ribonucleoside catabolic process [GO:0046130] Also known as: inosine breakdown, inosine catabolism, inosine degradation